{
  "term_label": "galanin-activated signaling pathway",
  "gene_name": "Galanin receptor type 3",
  "gene": "UniProtKB:O60755",
  "term_id": "GO:0090663",
  "gene_symbol": "GALR3"
}